{
  "gene": "UniProtKB:Q13519",
  "gene_name": "Prepronociceptin",
  "term_id": "GO:0005886",
  "term_label": "plasma membrane",
  "gene_symbol": "PNOC"
}